cyclomaltodextrin glucanotransferase activity [GO:0043895] (molecular function) Also known as: cyclodextrin glucanotransferase, 1,4-alpha-D-glucan 4-alpha-D-(1,4-alpha-D-glucano)-transferase (cyclizing), BMA, Bacillus macerans amylase, CGTase, alpha-1,4-glucan 4-glycosyltransferase, cyclizing, alpha-cyclodextrin glucanotransferase, alpha-cyclodextrin glycosyltransferase, beta-cyclodextrin glucanotransferase, beta-cyclodextrin glycosyltransferase, cyclodextrin glycosyltransferase, cyclomaltodextrin glucotransferase, cyclomaltodextrin glycosyltransferase, gamma-cyclodextrin glycosyltransferase, konchizaimu, neutral-cyclodextrin glycosyltransferase Sources: EC:2.4.1.19 Definition: Catalysis of the cyclization of part of a 1,4-alpha-D-glucan chain by formation of a 1,4-alpha-D-glucosidic bond. Relationships: is a type of hexosyltransferase activity [GO:0016758]